positive regulation of terrequinone A biosynthetic process [GO:1900854] (biological process) References: PMID:24066102 Sources: GOC:TermGenie, GOC:di Relationships: is a type of regulation of ketone biosynthetic process [GO:0010566]; is a type of positive regulation of small molecule metabolic process [GO:0062013]; is a type of GO:1900378; positively regulates GO:1900796 Definition: Any process that activates or increases the frequency, rate or extent of terrequinone A biosynthetic process. Also known as: regulation of terrequinone A biosynthetic process, up regulation of terrequinone A biosynthetic process, up-regulation of terrequinone A biosynthetic process, upregulation of terrequinone A biosynthetic process